{
  "gene": "UniProtKB:Q8WVM0",
  "term_label": "mitochondrial matrix",
  "term_id": "GO:0005759",
  "gene_name": "Dimethyladenosine transferase 1, mitochondrial",
  "gene_symbol": "TFB1M"
}